Group II intron splicing [GO:0000373] (biological process) Definition: The splicing of Group II introns. This occurs by a ribozymic mechanism where the intron sequence forms a distinct 3D structure, characteristic of Group II introns and containing splice site consensus sequences, that is involved in catalyzing the splicing reactions, though protein factors are also required in vivo. Splicing occurs by a series of two transesterification reactions (mechanistically similar to those for splicing of nuclear mRNAs) initiated by a bulged adenosine residue within the intron sequence as the initiating nucleophile. The intron is excised as a lariat. References: PMID:11377794 Sources: GOC:krc Also known as: mRNA splicing Note: Note that Group II introns are known to be found in a number of places: rRNA, mRNA, and tRNA in organelles of fungi, plants, and protists; and mRNA of bacteria. Relationships: is a type of GO:0000377